{
  "gene_name": "T cell receptor alpha joining 7 (Fragment)",
  "term_label": "Unknown biological process",
  "gene_symbol": "TRAJ7",
  "gene": "UniProtKB:A0A075B714",
  "term_id": "UNKNOWN:0002"
}